{
  "gene_name": "Nuclear receptor subfamily 4 group A member 3",
  "gene_symbol": "NR4A3",
  "term_id": "GO:0000978",
  "gene": "UniProtKB:Q92570",
  "term_label": "RNA polymerase II cis-regulatory region sequence-specific DNA binding"
}